riboflavin reductase (NADPH) activity [GO:0042602] (molecular function) Also known as: riboflavin mononucleotide reductase activity, riboflavine mononucleotide reductase activity, NADPH-riboflavin oxidoreductase activity, FMN reductase (NADPH) activity, NADPH dehydrogenase (riboflavin) activity, NADPH-FMN reductase activity, NADPH-dependent FMN reductase activity, NADPH-riboflavin reductase activity, NADPH-specific FMN reductase activity, NADPH:riboflavin oxidoreductase activity, flavin reductase activity, reduced-riboflavin:NADP+ oxidoreductase activity, riboflavin mononucleotide (reduced nicotinamide adenine dinucleotide phosphate) reductase activity Definition: Catalysis of the reaction: reduced riboflavin + NADP+ = riboflavin + NADPH + 2 H+. Relationships: is a type of riboflavin reductase [NAD(P)H] activity [GO:0052875] Sources: RHEA:19377